peptidyl-lysine trimethylation [GO:0018023] (biological process) Relationships: is a type of peptidyl-lysine methylation [GO:0018022] Sources: RESID:AA0074 Definition: The methylation of peptidyl-lysine to form peptidyl-N6,N6,N6-trimethyl-L-lysine.